{
  "term_label": "ribosomal large subunit biogenesis",
  "term_id": "GO:0042273",
  "gene": "UniProtKB:Q9BZE4",
  "gene_symbol": "GTPBP4",
  "gene_name": "GTP-binding protein 4"
}